post-transcriptional tethering of RNA polymerase II gene DNA at nuclear periphery [GO:0000973] (biological process) References: PMID:17373856, PMID:18614049 Sources: GOC:krc Relationships: is a type of transcription-dependent tethering of RNA polymerase II gene DNA at nuclear periphery [GO:0000972] Also known as: posttranscriptional tethering of RNA polymerase II gene DNA at nuclear periphery Definition: The chromosome organization process in which the DNA sequence containing a gene transcribed by RNA polymerase II is maintained in a specific location at the nuclear periphery even after transcription has been repressed.